{
  "term_label": "Unknown molecular function",
  "gene_name": "Olfactomedin-like protein 2A",
  "term_id": "UNKNOWN:0001",
  "gene_symbol": "OLFML2A",
  "gene": "UniProtKB:Q68BL7"
}